{
  "term_id": "GO:0006955",
  "gene_name": "Immunoglobulin kappa variable 1_OR2-108 (non-functional) (Fragment)",
  "gene_symbol": "IGKV1OR2-108",
  "gene": "UniProtKB:A0A075B7D4",
  "term_label": "immune response"
}